{
  "gene_symbol": "JUP",
  "gene": "UniProtKB:P14923",
  "term_id": "GO:0005737",
  "gene_name": "Junction plakoglobin",
  "term_label": "cytoplasm"
}